Leydig cell proliferation [GO:0160024] (biological process) References: PMID:29632025 Definition: The multiplication or reproduction of Leydig cells, resulting in the expansion of a cell population. Leydig cells are interstitial cells located adjacent to the seminiferous tubules in the testis which produce testosterone. Relationships: is a type of cell population proliferation [GO:0008283]